{
  "gene": "UniProtKB:Q8IU57",
  "term_id": "GO:0005886",
  "gene_name": "Interferon lambda receptor 1",
  "gene_symbol": "IFNLR1",
  "term_label": "plasma membrane"
}